{
  "gene_name": "Solute carrier family 13 member 2",
  "term_label": "cellular response to lithium ion",
  "term_id": "GO:0071285",
  "gene_symbol": "SLC13A2",
  "gene": "UniProtKB:Q13183"
}